{
  "term_id": "GO:0000307",
  "gene_name": "G1_S-specific cyclin-D2",
  "term_label": "cyclin-dependent protein kinase holoenzyme complex",
  "gene_symbol": "CCND2",
  "gene": "UniProtKB:P30279"
}